{
  "term_label": "ubiquitin protein ligase activity",
  "gene_symbol": "PJA2",
  "gene": "UniProtKB:O43164",
  "term_id": "GO:0061630",
  "gene_name": "E3 ubiquitin-protein ligase Praja-2"
}